{
  "gene_name": "A-kinase anchor protein 3",
  "gene_symbol": "AKAP3",
  "gene": "UniProtKB:O75969",
  "term_label": "sperm principal piece",
  "term_id": "GO:0097228"
}